peptidyl-lysine N6-myristoyltransferase activity [GO:0018030] (MF) Definition: Catalysis of the transfer of a myristoyl group to the N6 nitrogen atom on a lysine residue of a peptide or protein molecule. Relationships: is a type of myristoyltransferase activity [GO:0019107]; is a type of catalytic activity, acting on a protein [GO:0140096] Subtypes: ACP-dependent peptidyl-lysine N6-myristoyltransferase activity [GO:0140769], CoA-dependent peptidyl-lysine N6-myristoyltransferase activity [GO:0140770] References: PMID:1402651 Sources: GOC:mah